cellular response to peptide [GO:1901653] (biological process) Definition: Any process that results in a change in state or activity of a cell (in terms of movement, secretion, enzyme production, gene expression, etc.) as a result of a peptide stimulus. Relationships: is a type of cellular response to chemical stimulus [GO:0070887]; is_a response to peptide [GO:1901652] Sources: GOC:TermGenie, GOC:pr